{
  "term_label": "extracellular space",
  "gene_symbol": "C1QL1",
  "gene_name": "C1q-related factor",
  "term_id": "GO:0005615",
  "gene": "UniProtKB:O75973"
}